iodide transmembrane transporter activity [GO:0015111] (molecular function) Sources: GOC:ai Subtypes: sodium:iodide symporter activity [GO:0008507], GO:0160081 Relationships: is a type of GO:0008509; is part of iodide transport [GO:0015705] Definition: Enables the transfer of iodide ions from one side of a membrane to the other.